(+)-beta-barbatene synthase activity [GO:0102881] (molecular function) Relationships: is_a GO:0016838 References: PMID:15918888, PMID:16297850 Sources: RHEA:73983 Definition: Catalysis of the reaction: (2E,6E)-farnesyl diphosphate = (-)-beta-barbatene + diphosphate.